3-demethoxyubiquinol 3-hydroxylase activity [GO:0008682] (molecular function) Definition: Catalysis of the reaction: a 6-methoxy-3-methyl-2-all-trans-polyprenyl-1,4-benzoquinol + donor-H2 + O2 = acceptor + a 3-demethylubiquinol + H2O. Relationships: is a type of monooxygenase activity [GO:0004497]; is a type of oxidoreductase activity, acting on paired donors, with incorporation or reduction of molecular oxygen [GO:0016705] Sources: RHEA:50908 Also known as: 2-octoprenyl-3-methyl-6-methoxy-1,4-benzoquinone hydroxylase activity, demethoxy-ubiquinone hydroxylase, demethoxyubiquinone monooxygenase